response to granulocyte colony-stimulating factor [GO:1990638] (biological process) References: PMID:9488469 Also known as: response to G-CSF Relationships: is a type of GO:0034097 Definition: Any process that results in a change in state or activity of a cell or an organism (in terms of movement, secretion, enzyme production, gene expression, etc.) as a result of a granulocyte colony-stimulating factor stimulus. Subtypes: GO:1990643